{
  "term_label": "calcium-dependent phospholipid binding",
  "gene_symbol": "ESYT1",
  "gene": "UniProtKB:Q9BSJ8",
  "term_id": "GO:0005544",
  "gene_name": "Extended synaptotagmin-1"
}